{
  "gene": "UniProtKB:Q494U1",
  "gene_symbol": "PLEKHN1",
  "term_id": "GO:0061158",
  "term_label": "3'-UTR-mediated mRNA destabilization",
  "gene_name": "Pleckstrin homology domain-containing family N member 1"
}